quinoline-4-carboxylate 2-oxidoreductase activity [GO:0047123] (MF) Definition: Catalysis of the reaction: A + H2O + quinoline-4-carboxylate = 2-oxo-1,2-dihydroquinoline-4-carboxylate + AH(2). Sources: EC:1.3.99.19, RHEA:14949 Also known as: quinoline-4-carboxylate:acceptor 2-oxidoreductase (hydroxylating), quinoline-4-carboxylic acid 2-oxidoreductase activity Relationships: is a type of oxidoreductase activity, acting on the CH-CH group of donors [GO:0016627]